{
  "gene_symbol": "UAP1",
  "gene_name": "UDP-N-acetylhexosamine pyrophosphorylase",
  "gene": "UniProtKB:Q16222",
  "term_label": "UDP-N-acetylglucosamine diphosphorylase activity",
  "term_id": "GO:0003977"
}